{
  "term_label": "double-stranded DNA binding",
  "term_id": "GO:0003690",
  "gene": "UniProtKB:Q96B01",
  "gene_symbol": "RAD51AP1",
  "gene_name": "RAD51-associated protein 1"
}